{
  "term_id": "GO:0009897",
  "gene_name": "Asialoglycoprotein receptor 1",
  "gene_symbol": "ASGR1",
  "term_label": "external side of plasma membrane",
  "gene": "UniProtKB:P07306"
}